{
  "term_label": "microfibril binding",
  "gene_name": "Latent-transforming growth factor beta-binding protein 2",
  "gene": "UniProtKB:Q14767",
  "gene_symbol": "LTBP2",
  "term_id": "GO:0050436"
}